{
  "gene_symbol": "PITHD1",
  "term_label": "nucleus",
  "term_id": "GO:0005634",
  "gene": "UniProtKB:Q9GZP4",
  "gene_name": "PITH domain-containing protein 1"
}